{
  "gene_name": "Olfactory receptor 5H8",
  "gene_symbol": "OR5H8",
  "term_id": "GO:0005549",
  "term_label": "odorant binding",
  "gene": "UniProtKB:P0DN80"
}